{
  "term_label": "DNA binding",
  "gene_name": "Tigger transposable element-derived protein 5",
  "gene": "UniProtKB:Q53EQ6",
  "gene_symbol": "TIGD5",
  "term_id": "GO:0003677"
}